{
  "gene_name": "Immunoglobulin lambda variable 3-16",
  "gene_symbol": "IGLV3-16",
  "gene": "UniProtKB:A0A075B6K0",
  "term_id": "UNKNOWN:0001",
  "term_label": "Unknown molecular function"
}